uracil metabolic process [GO:0019860] (biological process) Definition: The chemical reactions and pathways involving uracil, 2,4-dioxopyrimidine, one of the pyrimidine bases occurring in RNA, but not in DNA. Sources: GOC:go_curators Also known as: uracil metabolism Relationships: is a type of pyrimidine nucleobase metabolic process [GO:0006206] Subtypes: uracil catabolic process [GO:0006212], uracil biosynthetic process [GO:0046107]